{
  "gene_symbol": "OR8D1",
  "term_id": "GO:0007608",
  "term_label": "sensory perception of smell",
  "gene_name": "Olfactory receptor 8D1",
  "gene": "UniProtKB:Q8WZ84"
}